{
  "term_label": "response to lipopolysaccharide",
  "term_id": "GO:0032496",
  "gene_name": "Protein S100-A8",
  "gene_symbol": "S100A8",
  "gene": "UniProtKB:P05109"
}